{
  "term_label": "Unknown cellular component",
  "term_id": "UNKNOWN:0003",
  "gene_name": "C2 calcium-dependent domain-containing protein 4D",
  "gene": "UniProtKB:B7Z1M9",
  "gene_symbol": "C2CD4D"
}